{
  "term_label": "Unknown biological process",
  "gene": "UniProtKB:Q5VZV1",
  "gene_name": "Protein-lysine methyltransferase METTL21C",
  "term_id": "UNKNOWN:0002",
  "gene_symbol": "METTL21C"
}